keto-D-gluconate biosynthetic process [GO:0046179] (biological process) Also known as: keto-D-gluconate anabolism, keto-D-gluconate biosynthesis, keto-D-gluconate formation, keto-D-gluconate synthesis Definition: The chemical reactions and pathways resulting in the formation of keto-D-gluconate, the anion of keto-D-gluconic acid, an aldonic acid derived from glucose. Sources: ISBN:0198506732 Relationships: is_a ketogluconate biosynthetic process [GO:0046180]